{
  "term_label": "Unknown biological process",
  "term_id": "UNKNOWN:0002",
  "gene_name": "Mediator of RNA polymerase II transcription subunit 28",
  "gene_symbol": "MED28",
  "gene": "UniProtKB:Q9H204"
}